{
  "gene_symbol": "FHIP1A",
  "gene": "UniProtKB:Q05DH4",
  "term_id": "UNKNOWN:0002",
  "gene_name": "FHF complex subunit HOOK-interacting protein 1A",
  "term_label": "Unknown biological process"
}